regulation of t-circle formation [GO:1904429] (biological process) Relationships: is a type of GO:0032204; is_a regulation of cellular component biogenesis [GO:0044087]; regulates GO:0090656 Definition: Any process that modulates the frequency, rate or extent of t-circle formation. Subtypes: GO:1904430, positive regulation of t-circle formation [GO:1904431] Also known as: regulation of telomeric circle formation References: PMID:22579284 Sources: GOC:BHF, GOC:BHF_telomere, GOC:TermGenie, GOC:nc, GO_REF:0000058